{
  "gene_symbol": "CEP20",
  "gene_name": "Centrosomal protein 20",
  "term_label": "motile cilium",
  "gene": "UniProtKB:Q96NB1",
  "term_id": "GO:0031514"
}